{
  "term_label": "nucleus",
  "gene": "UniProtKB:O15522",
  "gene_symbol": "NKX2-8",
  "term_id": "GO:0005634",
  "gene_name": "Homeobox protein Nkx-2.8"
}